{
  "term_label": "Unknown biological process",
  "gene_symbol": "CCDC71",
  "gene": "UniProtKB:Q8IV32",
  "term_id": "UNKNOWN:0002",
  "gene_name": "Coiled-coil domain-containing protein 71"
}